L-beta-ethynylserine biosynthetic process [GO:0062142] (biological process) Definition: The chemical reactions and pathways resulting in the formation of L-beta-ethynylserine. L-beta-ethynylserine is an antibiotic produced by Streptomyces bacteria. Relationships: is a type of L-amino acid biosynthetic process [GO:0170034]; is a type of non-proteinogenic amino acid biosynthetic process [GO:0170043] References: PMID:3082841, PMID:30867596